{
  "term_label": "Unknown molecular function",
  "term_id": "UNKNOWN:0001",
  "gene_symbol": "WDR24",
  "gene_name": "GATOR complex protein WDR24",
  "gene": "UniProtKB:Q96S15"
}